negative regulation of protein targeting to mitochondrion [GO:1903215] (biological process) References: PMID:21370995 Sources: GOC:PARL, GOC:TermGenie, GOC:bf, GO_REF:0000058 Also known as: down regulation of protein import into mitochondrion, down regulation of protein targeting to mitochondria, down regulation of protein targeting to mitochondrion, down regulation of protein-mitochondrial targeting, down-regulation of protein import into mitochondrion, down-regulation of protein targeting to mitochondria, down-regulation of protein targeting to mitochondrion, down-regulation of protein-mitochondrial targeting, downregulation of protein import into mitochondrion, downregulation of protein targeting to mitochondria, downregulation of protein targeting to mitochondrion, downregulation of protein-mitochondrial targeting, negative regulation of protein import into mitochondrion, negative regulation of protein targeting to mitochondria, negative regulation of protein-mitochondrial targeting, inhibition of protein import into mitochondrion, inhibition of protein targeting to mitochondria, inhibition of protein targeting to mitochondrion, inhibition of protein-mitochondrial targeting, down regulation of mitochondrial protein import, down regulation of mitochondrial translocation, down-regulation of mitochondrial protein import, down-regulation of mitochondrial translocation, downregulation of mitochondrial protein import, downregulation of mitochondrial translocation, inhibition of mitochondrial protein import, inhibition of mitochondrial translocation, negative regulation of mitochondrial protein import, negative regulation of mitochondrial translocation Definition: Any process that stops, prevents or reduces the frequency, rate or extent of protein targeting to mitochondrion. Subtypes: negative regulation of protein insertion into mitochondrial outer membrane [GO:1903637] Relationships: is a type of regulation of protein targeting to mitochondrion [GO:1903214]; is a type of negative regulation of establishment of protein localization to mitochondrion [GO:1903748]; negatively regulates protein targeting to mitochondrion [GO:0006626]